{
  "gene_name": "Protein bicaudal D homolog 1",
  "term_label": "cytosol",
  "gene_symbol": "BICD1",
  "term_id": "GO:0005829",
  "gene": "UniProtKB:Q96G01"
}